{
  "term_id": "GO:0022627",
  "gene_symbol": "RPS17",
  "term_label": "cytosolic small ribosomal subunit",
  "gene": "UniProtKB:P08708",
  "gene_name": "Small ribosomal subunit protein eS17"
}